{
  "gene": "UniProtKB:A5YM72",
  "gene_name": "Carnosine synthase 1",
  "term_id": "GO:0035499",
  "term_label": "carnosine biosynthetic process",
  "gene_symbol": "CARNS1"
}